{
  "gene_name": "DNA polymerase lambda",
  "gene": "UniProtKB:Q9UGP5",
  "gene_symbol": "POLL",
  "term_label": "double-strand break repair via nonhomologous end joining",
  "term_id": "GO:0006303"
}